{
  "term_id": "GO:0005576",
  "gene_name": "EGF-containing fibulin-like extracellular matrix protein 1",
  "gene_symbol": "EFEMP1",
  "gene": "UniProtKB:Q12805",
  "term_label": "extracellular region"
}